{
  "gene_name": "Casein kinase I isoform epsilon",
  "gene_symbol": "CSNK1E",
  "term_label": "positive regulation of canonical Wnt signaling pathway",
  "gene": "UniProtKB:P49674",
  "term_id": "GO:0090263"
}